{
  "term_id": "GO:0000978",
  "gene_symbol": "BHLHE40",
  "gene": "UniProtKB:O14503",
  "gene_name": "Class E basic helix-loop-helix protein 40",
  "term_label": "RNA polymerase II cis-regulatory region sequence-specific DNA binding"
}